3-deoxy-8-phosphooctulonate synthase activity [GO:0008676] (molecular function) Relationships: is a type of transferase activity, transferring alkyl or aryl (other than methyl) groups [GO:0016765] Sources: EC:2.5.1.55, RHEA:14053 Also known as: 2-dehydro-3-deoxyphosphooctonate aldolase activity, 2-dehydro-3-deoxy-D-octonate-8-phosphate D-arabinose-5-phosphate-lyase (pyruvate-phosphorylating) activity, 2-dehydro-3-deoxy-phosphooctonate aldolase activity, 2-keto-3-deoxy-8-phosphooctonic synthetase activity, 3-deoxy-D-manno-octulosonate-8-phosphate synthase activity, 3-deoxy-D-manno-octulosonic acid 8-phosphate synthetase activity, 3-deoxy-D-mannooctulosonate-8-phosphate synthetase activity, 3-deoxyoctulosonic 8-phosphate synthetase activity, KDO-8-P synthase activity, KDO-8-phosphate synthetase activity, KDOP synthase activity, phospho-2-keto-3-deoxyoctonate aldolase activity, phosphoenolpyruvate:D-arabinose-5-phosphate C-(1-carboxyvinyl)transferase (phosphate-hydrolysing, 2-carboxy-2-oxoethyl-forming) Definition: Catalysis of the reaction: D-arabinose 5-phosphate + H2O + phosphoenolpyruvate = 8-phospho-3-deoxy-D-manno-oct-2-ulosonate + 2 H+ + phosphate.